{
  "term_id": "GO:0008020",
  "gene": "UniProtKB:O14718",
  "gene_symbol": "RRH",
  "term_label": "G protein-coupled photoreceptor activity",
  "gene_name": "Visual pigment-like receptor peropsin"
}